{
  "gene_symbol": "FER1L6",
  "gene_name": "Fer-1-like protein 6",
  "term_label": "positive regulation of gene expression",
  "gene": "UniProtKB:Q2WGJ9",
  "term_id": "GO:0010628"
}